{
  "gene_name": "C-C motif chemokine 20",
  "gene_symbol": "CCL20",
  "term_label": "Unknown cellular component",
  "gene": "UniProtKB:P78556",
  "term_id": "UNKNOWN:0003"
}